{
  "term_id": "GO:0005829",
  "gene_name": "NAD-dependent protein deacylase sirtuin-5, mitochondrial",
  "gene_symbol": "SIRT5",
  "term_label": "cytosol",
  "gene": "UniProtKB:Q9NXA8"
}